{
  "gene_symbol": "RIN2",
  "gene": "UniProtKB:Q8WYP3",
  "term_id": "UNKNOWN:0002",
  "term_label": "Unknown biological process",
  "gene_name": "Ras and Rab interactor 2"
}